progression of morphogenetic furrow involved in compound eye morphogenesis [GO:0007458] (biological process) Definition: The morphogenetic furrow is a dorsoventral indentation which sweeps anteriorly across the eye disc. Ommatidia begin to form along the furrow, resulting in a graded series of ommatidial development across the anterior/posterior axis of the disc. Relationships: is a type of anatomical structure development [GO:0048856]; is part of GO:0001745 Also known as: progression of morphogenetic furrow during compound eye morphogenesis References: PMID:3076112, PMID:3937883